{
  "gene": "UniProtKB:P78540",
  "gene_symbol": "ARG2",
  "term_id": "GO:0005737",
  "term_label": "cytoplasm",
  "gene_name": "Arginase-2, mitochondrial"
}